{
  "term_id": "GO:0051603",
  "gene": "UniProtKB:P43235",
  "term_label": "proteolysis involved in protein catabolic process",
  "gene_name": "Cathepsin K",
  "gene_symbol": "CTSK"
}